terpenoid indole alkaloid metabolic process [GO:0046447] (biological process) Also known as: terpenoid indole alkaloid metabolism Definition: The chemical reactions and pathways involving terpenoid indole alkaloids, compounds formed from the condensation of tryptamine (derived from tryptophan) and secologanin (derived from geranyl pyrophosphate). Subtypes: terpenoid indole alkaloid biosynthetic process [GO:0009709] Relationships: is a type of GO:0035834 Sources: GOC:ai